{
  "term_id": "GO:0031209",
  "gene_name": "Actin-binding protein WASF1",
  "term_label": "SCAR complex",
  "gene_symbol": "WASF1",
  "gene": "UniProtKB:Q92558"
}